{
  "gene": "UniProtKB:Q7L4S7",
  "term_label": "mitochondrion",
  "gene_name": "Protein ARMCX6",
  "gene_symbol": "ARMCX6",
  "term_id": "GO:0005739"
}